positive regulation of pancreatic stellate cell proliferation [GO:2000231] (BP) Sources: GOC:mah Relationships: is a type of positive regulation of fibroblast proliferation [GO:0048146]; is a type of regulation of pancreatic stellate cell proliferation [GO:2000229]; positively regulates pancreatic stellate cell proliferation [GO:0072343] Definition: Any process that activates or increases the frequency, rate or extent of pancreatic stellate cell proliferation.